{
  "gene": "UniProtKB:P61019",
  "gene_name": "Ras-related protein Rab-2A",
  "term_id": "GO:0016192",
  "gene_symbol": "RAB2A",
  "term_label": "vesicle-mediated transport"
}